{
  "term_id": "GO:0071035",
  "gene_name": "Exosome component 10",
  "gene_symbol": "EXOSC10",
  "gene": "UniProtKB:Q01780",
  "term_label": "nuclear polyadenylation-dependent rRNA catabolic process"
}